{
  "gene_symbol": "IGHV1-24",
  "term_id": "GO:0003823",
  "gene": "UniProtKB:A0A0C4DH33",
  "gene_name": "Immunoglobulin heavy variable 1-24",
  "term_label": "antigen binding"
}